{
  "gene_name": "Transcription factor SOX-4",
  "gene_symbol": "SOX4",
  "gene": "UniProtKB:Q06945",
  "term_label": "positive regulation of transcription by RNA polymerase II",
  "term_id": "GO:0045944"
}